{
  "gene": "UniProtKB:A0A577",
  "term_label": "Unknown molecular function",
  "gene_name": "T cell receptor beta variable 4-1",
  "term_id": "UNKNOWN:0001",
  "gene_symbol": "TRBV4-1"
}